B cell activation [GO:0042113] (BP) Sources: GOC:mgi_curators, ISBN:0781735149 Regulation: regulated by regulation of B cell activation [GO:0050864]; negatively regulated by negative regulation of B cell activation [GO:0050869]; positively regulated by positive regulation of B cell activation [GO:0050871] Also known as: B lymphocyte activation, B-cell activation, B-lymphocyte activation Relationships: is a type of lymphocyte activation [GO:0046649] Subtypes: B cell activation involved in immune response [GO:0002312], B cell differentiation [GO:0030183], GO:0042100 Definition: The change in morphology and behavior of a mature or immature B cell resulting from exposure to a mitogen, cytokine, chemokine, cellular ligand, or an antigen for which it is specific.